potassium ion homeostasis [GO:0055075] (biological process) Sources: GOC:jid, GOC:mah Subtypes: GO:0030007 Relationships: is a type of GO:0055080; is a type of inorganic ion homeostasis [GO:0098771] Definition: Any process involved in the maintenance of an internal steady state of potassium ions within an organism or cell.